lysosomal membrane organization [GO:0097212] (biological process) Definition: A process that is carried out at the cellular level which results in the assembly, arrangement of constituent parts, or disassembly of a lysosomal membrane. A lysosomal membrane is the lipid bilayer surrounding the lysosome and separating its contents from the cell cytoplasm. References: PMID:20544854 Sources: GOC:yaf Also known as: lysosomal membrane organisation, lysosome membrane organization Relationships: is a type of membrane organization [GO:0061024]; is part of lysosome organization [GO:0007040] Subtypes: multivesicular body-lysosome fusion [GO:0061763], regulation of lysosomal membrane permeability [GO:0097213]